{
  "term_id": "GO:0005886",
  "gene_name": "Transmembrane gamma-carboxyglutamic acid protein 2",
  "gene_symbol": "PRRG2",
  "term_label": "plasma membrane",
  "gene": "UniProtKB:O14669"
}